{
  "gene_name": "Cholinephosphotransferase 1",
  "gene": "UniProtKB:Q8WUD6",
  "gene_symbol": "CHPT1",
  "term_label": "endoplasmic reticulum membrane",
  "term_id": "GO:0005789"
}